{
  "gene_name": "Gap junction beta-1 protein",
  "term_id": "GO:0005922",
  "gene_symbol": "GJB1",
  "term_label": "connexin complex",
  "gene": "UniProtKB:P08034"
}